{
  "term_id": "GO:0016423",
  "gene_symbol": "TARBP1",
  "gene": "UniProtKB:Q13395",
  "term_label": "tRNA (guanine) methyltransferase activity",
  "gene_name": "Probable methyltransferase TARBP1"
}